{
  "gene_name": "Ras and Rab interactor-like protein",
  "gene_symbol": "RINL",
  "term_label": "Unknown biological process",
  "term_id": "UNKNOWN:0002",
  "gene": "UniProtKB:Q6ZS11"
}